{
  "term_id": "GO:0005813",
  "gene_symbol": "MPLKIP",
  "term_label": "centrosome",
  "gene": "UniProtKB:Q8TAP9",
  "gene_name": "M-phase-specific PLK1-interacting protein"
}